{
  "gene_name": "Twinfilin-1",
  "term_id": "GO:0010976",
  "gene_symbol": "TWF1",
  "term_label": "positive regulation of neuron projection development",
  "gene": "UniProtKB:Q12792"
}